{
  "term_id": "GO:0061631",
  "gene_symbol": "UBE2S",
  "gene": "UniProtKB:Q16763",
  "term_label": "ubiquitin conjugating enzyme activity",
  "gene_name": "Ubiquitin-conjugating enzyme E2 S"
}